{
  "gene_name": "Hepatocyte nuclear factor 3-alpha",
  "term_id": "GO:0006357",
  "gene": "UniProtKB:P55317",
  "term_label": "regulation of transcription by RNA polymerase II",
  "gene_symbol": "FOXA1"
}